{
  "term_id": "GO:0007274",
  "gene_name": "F-BAR and double SH3 domains protein 1",
  "gene": "UniProtKB:Q86WN1",
  "term_label": "neuromuscular synaptic transmission",
  "gene_symbol": "FCHSD1"
}